cis-Golgi network [GO:0005801] (cellular component) Definition: The network of interconnected tubular and cisternal structures located at the convex side of the Golgi apparatus, which abuts the endoplasmic reticulum. Note: The CGN is not considered part of the Golgi stack. Relationships: is a type of intracellular membrane-bounded organelle [GO:0043231]; is part of Golgi apparatus [GO:0005794] Also known as: cis face, cis Golgi network, Golgi cis face, Golgi cis-face, forming face References: PMID:23543640, PMID:9695800 Sources: ISBN:0198506732, ISBN:0815316194